{
  "term_id": "GO:0004000",
  "gene_symbol": "MAPDA",
  "gene": "UniProtKB:Q6DHV7",
  "term_label": "adenosine deaminase activity",
  "gene_name": "Adenosine deaminase-like protein"
}